{
  "gene": "UniProtKB:P55157",
  "gene_name": "Microsomal triglyceride transfer protein large subunit",
  "term_label": "lipoprotein metabolic process",
  "gene_symbol": "MTTP",
  "term_id": "GO:0042157"
}